{
  "gene_symbol": "SAMD5",
  "gene_name": "Sterile alpha motif domain-containing protein 5",
  "term_label": "Unknown molecular function",
  "term_id": "UNKNOWN:0001",
  "gene": "UniProtKB:Q5TGI4"
}